{
  "gene_symbol": "ST18",
  "term_label": "Unknown molecular function",
  "term_id": "UNKNOWN:0001",
  "gene_name": "Suppression of tumorigenicity 18 protein",
  "gene": "UniProtKB:O60284"
}